{
  "gene_symbol": "RHPN1-AS1",
  "gene": "UniProtKB:Q9BWJ2",
  "term_label": "Unknown biological process",
  "gene_name": "Putative uncharacterized protein encoded by RHPN1-AS1",
  "term_id": "UNKNOWN:0002"
}